{
  "gene_name": "GTPase KRas",
  "gene": "UniProtKB:P01116",
  "term_id": "GO:0005886",
  "term_label": "plasma membrane",
  "gene_symbol": "KRAS"
}